{
  "gene": "UniProtKB:Q16288",
  "term_id": "GO:0043235",
  "term_label": "receptor complex",
  "gene_name": "NT-3 growth factor receptor",
  "gene_symbol": "NTRK3"
}